cholesterol dehydrogenase (NAD+) activity [GO:0102294] (MF) Sources: RHEA:35459 Relationships: is a type of GO:0003854 Definition: Catalysis of the reaction: cholesterol + NAD+ = cholest-5-en-3-one + NADH + H+.